{
  "gene_name": "Small kinetochore-associated protein",
  "gene": "UniProtKB:Q9Y448",
  "gene_symbol": "KNSTRN",
  "term_label": "kinetochore",
  "term_id": "GO:0000776"
}